carnosine biosynthetic process [GO:0035499] (biological process) Definition: The chemical reactions and pathways resulting in the formation of the dipeptide beta-alanyl-L-histidine (carnosine). Also known as: carnosine anabolism, carnosine biosynthesis, carnosine formation, carnosine synthesis References: PMID:20097752 Relationships: is a type of amino acid biosynthetic process [GO:0008652]; is a type of carnosine metabolic process [GO:0035498]; is a type of GO:0043604; is a type of carboxylic acid biosynthetic process [GO:0046394]